positive regulation of protein localization to synapse [GO:1902474] (biological process) Definition: Any process that activates or increases the frequency, rate or extent of protein localization to synapse. Subtypes: positive regulation of protein localization to presynapse [GO:1905386] Also known as: positive regulation of protein localisation to synapse, up regulation of protein localisation to synapse, up regulation of protein localization to synapse, up-regulation of protein localisation to synapse, up-regulation of protein localization to synapse, upregulation of protein localisation to synapse, upregulation of protein localization to synapse, activation of protein localisation to synapse, activation of protein localization to synapse Relationships: is a type of regulation of protein localization to synapse [GO:1902473]; is_a positive regulation of protein localization [GO:1903829]; positively regulates GO:0035418 References: PMID:22588719 Sources: GOC:TermGenie, GOC:kmv